{
  "gene_name": "Ubiquitin-conjugating enzyme E2 R2",
  "term_label": "ubiquitin conjugating enzyme activity",
  "term_id": "GO:0061631",
  "gene_symbol": "UBE2R2",
  "gene": "UniProtKB:Q712K3"
}